membrane raft [GO:0045121] (CC) Definition: Any of the small (10-200 nm), heterogeneous, highly dynamic, sterol- and sphingolipid-enriched membrane domains that compartmentalize cellular processes. Small rafts can sometimes be stabilized to form larger platforms through protein-protein and protein-lipid interactions. References: PMID:16645198, PMID:20044567 Also known as: lipid raft, GEM domain, glycolipid-enriched membrane domain Relationships: is a type of membrane microdomain [GO:0098857] Subtypes: GO:0044853